{
  "gene_symbol": "CPNE6",
  "term_label": "cellular response to calcium ion",
  "gene": "UniProtKB:O95741",
  "gene_name": "Copine-6",
  "term_id": "GO:0071277"
}